{
  "term_id": "UNKNOWN:0002",
  "gene_symbol": "TMEM233",
  "gene": "UniProtKB:B4DJY2",
  "gene_name": "Transmembrane protein 233",
  "term_label": "Unknown biological process"
}